modified amino acid transport [GO:0072337] (biological process) Relationships: is a type of nitrogen compound transport [GO:0071705] Sources: GOC:mah Also known as: amino acid derivative transport Definition: The directed movement of modified amino acids into, out of or within a cell, or between cells, by means of some agent such as a transporter or pore. Subtypes: S-methylmethionine transport [GO:0015806], GO:0015811, p-aminobenzoyl-glutamate transport [GO:0015814], amino-acid betaine transport [GO:0015838], creatine transmembrane transport [GO:0015881], folic acid transport [GO:0015884], 5-formyltetrahydrofolate transport [GO:0015885], pantothenate transmembrane transport [GO:0015887], aerobactin transport [GO:0019271], hydroxyproline transport [GO:0034589], glutathione transport [GO:0034635], GO:1905130